{
  "gene": "UniProtKB:Q9BXJ8",
  "gene_name": "Ion channel TACAN",
  "term_id": "UNKNOWN:0001",
  "term_label": "Unknown molecular function",
  "gene_symbol": "TMEM120A"
}